maintenance of dauer [GO:0043055] (biological process) Definition: Maintenance of a nematode during the facultative diapause of the dauer (enduring) larval stage of nematode development. Relationships: is a type of GO:0071982; BFO_0000050 GO:0040024 Sources: GOC:cab1, WB_REF:wm2003ab740 Also known as: maintenance of dormancy in the nematode